hexasaccharide transport [GO:2001102] (biological process) Subtypes: maltohexaose transport [GO:2001103] Regulation: regulated by regulation of hexasaccharide transport [GO:1900297]; negatively regulated by negative regulation of hexasaccharide transport [GO:1900298]; positively regulated by GO:1900299 Definition: The directed movement of a hexasaccharideacetate into, out of or within a cell, or between cells, by means of some agent such as a transporter or pore. Relationships: is a type of GO:0015772 Sources: GOC:mengo_curators